{
  "term_id": "GO:0042910",
  "gene_name": "Multidrug and toxin extrusion protein 1",
  "gene_symbol": "SLC47A1",
  "term_label": "xenobiotic transmembrane transporter activity",
  "gene": "UniProtKB:Q96FL8"
}